{
  "gene_name": "Granulocyte-macrophage colony-stimulating factor receptor subunit alpha",
  "gene_symbol": "CSF2RA",
  "term_label": "external side of plasma membrane",
  "gene": "UniProtKB:P15509",
  "term_id": "GO:0009897"
}